glycoprotein 6-alpha-L-fucosyltransferase activity [GO:0008424] (molecular function) Also known as: glycoprotein fucosyltransferase activity, FucT, GDP-L-Fuc:N-acetyl-beta-D-glucosaminide alpha(1,6)fucosyltransferase activity, GDP-L-Fuc:N-acetyl-beta-D-glucosaminide alpha(1->6)fucosyltransferase activity, GDP-L-Fuc:N-acetyl-beta-D-glucosaminide alpha-(1,6)fucosyltransferase activity, GDP-L-Fuc:N-acetyl-beta-D-glucosaminide alpha-(1->6)fucosyltransferase activity, GDP-L-fucose--glycoprotein fucosyltransferase activity, GDP-fucose--glycoprotein fucosyltransferase activity, GDPfucose-glycoprotein fucosyltransferase activity, guanosine diphosphofucose--glycoprotein fucosyltransferase activity Relationships: is a type of GO:0046921; is a type of catalytic activity, acting on a glycoprotein [GO:0140103]; is part of protein O-linked glycosylation via fucose [GO:0036066] Definition: Catalysis of the reaction: N(4)-{N-acetyl-beta-D-glucosaminyl-(1->2)-alpha-D-mannosyl-(1->3)-[N-acetyl-beta-D-glucosaminyl-(1->2)-alpha-D-mannosyl-(1->6)]-beta-D-mannosyl-(1->4)-N-acetyl-beta-D-glucosaminyl-(1->4)-N-acetyl-beta-D-glucosaminyl}-L-asparagine + GDP-L-fucose = N(4)-{N-acetyl-beta-D-glucosaminyl-(1->2)-alpha-D-mannosyl-(1->3)-[N-acetyl-beta-D-glucosaminyl-(1->2)-alpha-D-mannosyl-(1->6)]-beta-D-mannosyl-(1->4)-N-acetyl-beta-D-glucosaminyl-(1->4)-[alpha-L-fucosyl-(1->6)]-N-acetyl-beta-D-glucosaminyl}asparagine + GDP + H+. Sources: EC:2.4.1.68, RHEA:12985